{
  "term_label": "synapse",
  "gene_name": "Synaptotagmin-7",
  "term_id": "GO:0045202",
  "gene": "UniProtKB:O43581",
  "gene_symbol": "SYT7"
}